{
  "gene_symbol": "RARB",
  "gene_name": "Retinoic acid receptor beta",
  "gene": "UniProtKB:P10826",
  "term_label": "negative regulation of transcription by RNA polymerase II",
  "term_id": "GO:0000122"
}